{
  "term_id": "GO:1904862",
  "gene_symbol": "GABRA1",
  "gene_name": "Gamma-aminobutyric acid receptor subunit alpha-1",
  "term_label": "inhibitory synapse assembly",
  "gene": "UniProtKB:P14867"
}